negative regulation of peripheral tolerance induction [GO:0002659] (biological process) Subtypes: GO:0002844, negative regulation of peripheral T cell tolerance induction [GO:0002850], GO:0002909, negative regulation of peripheral B cell anergy [GO:0002918] Relationships: is a type of negative regulation of tolerance induction dependent upon immune response [GO:0002653]; is a type of regulation of peripheral tolerance induction [GO:0002658]; negatively regulates peripheral tolerance induction [GO:0002465] Sources: GOC:add Also known as: down regulation of peripheral tolerance induction, down-regulation of peripheral tolerance induction, downregulation of peripheral tolerance induction, inhibition of peripheral tolerance induction Definition: Any process that stops, prevents, or reduces the frequency, rate, or extent of peripheral tolerance induction.